N-ethylmaleimide reductase activity [GO:0008748] (molecular function) Sources: MetaCyc:RXN0-5101 Relationships: is a type of oxidoreductase activity, acting on the CH-CH group of donors, NAD or NADP as acceptor [GO:0016628] Definition: Catalysis of the reaction: N-ethylmaleimide + NADPH + 2 H+ = N-ethylsuccinimide + NADP+.